{
  "term_id": "GO:0006897",
  "gene_name": "Endophilin-A2",
  "term_label": "endocytosis",
  "gene": "UniProtKB:Q99961",
  "gene_symbol": "SH3GL1"
}